{
  "term_label": "lumenal side of endoplasmic reticulum membrane",
  "gene": "UniProtKB:Q8IUH8",
  "term_id": "GO:0098553",
  "gene_name": "Signal peptide peptidase-like 2C",
  "gene_symbol": "SPPL2C"
}